{
  "gene": "UniProtKB:O95863",
  "term_id": "GO:0000978",
  "term_label": "RNA polymerase II cis-regulatory region sequence-specific DNA binding",
  "gene_symbol": "SNAI1",
  "gene_name": "Zinc finger protein SNAI1"
}